{
  "gene": "UniProtKB:P11021",
  "gene_symbol": "HSPA5",
  "term_id": "GO:0030968",
  "gene_name": "Endoplasmic reticulum chaperone BiP",
  "term_label": "endoplasmic reticulum unfolded protein response"
}